G protein-coupled olfactory receptor activity [GO:0038022] (molecular function) Definition: Combining with an odorant and transmitting the signal across the membrane by activating an associated G-protein; promotes the exchange of GDP for GTP on the alpha subunit of a heterotrimeric G-protein complex. Also known as: G-protein coupled odorant receptor activity, G-protein coupled olfactory receptor activity, olfactory receptor activity, G-protein coupled, odorant receptor activity, G-protein coupled References: PMID:21041441 Sources: GOC:bf, GOC:sart Relationships: is a type of G protein-coupled receptor activity [GO:0004930]; is a type of olfactory receptor activity [GO:0004984]